{
  "term_id": "UNKNOWN:0003",
  "gene_name": "Post-GPI attachment to proteins factor 3",
  "gene": "UniProtKB:Q96FM1",
  "term_label": "Unknown cellular component",
  "gene_symbol": "PGAP3"
}